negative regulation of the force of heart contraction involved in baroreceptor response to increased systemic arterial blood pressure [GO:0001986] (biological process) Sources: GOC:mtg_cardio, ISBN:0721643949 Definition: Any process that decreases the force with which the cardiac muscles of the heart pump blood through the circulatory system as a result of the baroreceptor response to increased blood pressure. Relationships: is a type of negative regulation of heart contraction [GO:0045822]; is part of baroreceptor response to increased systemic arterial blood pressure [GO:0001983] Also known as: decreased force of heart contraction during baroreceptor response to increased systemic arterial blood pressure, decreased strength of cardiac contraction during baroreceptor response to increased blood pressure